G protein-coupled receptor signaling pathway [GO:0007186] (biological process) Subtypes: sphingosine-1-phosphate receptor signaling pathway [GO:0003376], GO:0007187, GO:0007188, phospholipase C-activating G protein-coupled receptor signaling pathway [GO:0007200], octopamine or tyramine signaling pathway [GO:0007211], G protein-coupled dopamine receptor signaling pathway [GO:0007212], G protein-coupled acetylcholine receptor signaling pathway [GO:0007213], G protein-coupled glutamate receptor signaling pathway [GO:0007216], tachykinin receptor signaling pathway [GO:0007217], neuropeptide signaling pathway [GO:0007218], G protein-coupled opsin signaling pathway [GO:0016056], GO:0030845, phospholipase D-activating G protein-coupled receptor signaling pathway [GO:0031583], bombesin receptor signaling pathway [GO:0031989], G protein-coupled purinergic receptor signaling pathway [GO:0035588], G protein-coupled opioid receptor signaling pathway [GO:0038003], angiotensin-activated signaling pathway [GO:0038166], somatostatin receptor signaling pathway [GO:0038169], cannabinoid signaling pathway [GO:0038171], complement component C5a signaling pathway [GO:0038178], GO:0038188, gastric inhibitory peptide signaling pathway [GO:0038192], thromboxane A2 signaling pathway [GO:0038193], thyroid-stimulating hormone signaling pathway [GO:0038194], follicle-stimulating hormone signaling pathway [GO:0042699], GO:0042700, apelin receptor signaling pathway [GO:0060183], leukotriene signaling pathway [GO:0061737], chemokine-mediated signaling pathway [GO:0070098], GO:0070493, GO:0071875, endothelin receptor signaling pathway [GO:0086100], G protein-coupled receptor signaling pathway involved in heart process [GO:0086103], calcitonin family receptor signaling pathway [GO:0097646], G protein-coupled serotonin receptor signaling pathway [GO:0098664], G protein-coupled chemorepellent receptor signaling pathway [GO:0140986], Rho-activating G protein-coupled receptor signaling pathway [GO:0160221], G protein-coupled receptor signaling pathway involved in defense response to Gram-negative bacterium [GO:1903554], GO:1904066, G protein-coupled receptor signaling pathway involved in social behavior [GO:1904068] Also known as: G protein coupled receptor protein signaling pathway, G protein coupled receptor protein signalling pathway, G-protein coupled receptor protein signal transduction, G-protein coupled receptor protein signaling pathway, G-protein coupled receptor signalling pathway, G-protein-coupled receptor protein signalling pathway, GPCR signaling pathway, GPCR signalling pathway, G-protein coupled receptor signaling pathway via GPCR dimer, dimeric G-protein coupled receptor signaling pathway, dimeric G-protein coupled receptor signalling pathway Definition: The series of molecular signals initiated by a ligand binding to its receptor, in which the activated receptor promotes the exchange of GDP for GTP on the alpha-subunit of an associated heterotrimeric G-protein complex. The GTP-bound activated alpha-G-protein then dissociates from the beta- and gamma-subunits to further transmit the signal within the cell. The pathway begins with receptor-ligand interaction, and ends with regulation of a downstream cellular process. The pathway can start from the plasma membrane, Golgi or nuclear membrane. Regulation: regulated by regulation of G protein-coupled receptor signaling pathway [GO:0008277]; negatively regulated by negative regulation of G protein-coupled receptor signaling pathway [GO:0045744]; positively regulated by GO:0045745 Relationships: is a type of signal transduction [GO:0007165]; has part G protein-coupled receptor activity [GO:0004930] References: PMID:16902576, PMID:24568158 Sources: GOC:bf, GOC:mah, Wikipedia:G_protein-coupled_receptor